{
  "term_label": "dendrite membrane",
  "gene_symbol": "AKAP5",
  "term_id": "GO:0032590",
  "gene": "UniProtKB:P24588",
  "gene_name": "A-kinase anchor protein 5"
}